voltage-gated potassium channel activity [GO:0005249] (MF) Definition: Enables the transmembrane transfer of a potassium ion by a voltage-gated channel. A voltage-gated channel is a channel whose open state is dependent on the voltage across the membrane in which it is embedded. Sources: GOC:mtg_transport, ISBN:0815340729 Also known as: voltage gated potassium channel activity, voltage-dependent potassium channel activity, voltage-gated potassium ion channel activity, voltage-sensitive potassium channel Relationships: is a type of potassium channel activity [GO:0005267]; is a type of voltage-gated monoatomic cation channel activity [GO:0022843] Subtypes: GO:0005242, delayed rectifier potassium channel activity [GO:0005251], open rectifier potassium channel activity [GO:0005252], outward rectifier potassium channel activity [GO:0015271], voltage-gated potassium channel activity involved in cardiac muscle cell action potential repolarization [GO:0086008], voltage-gated potassium channel activity involved in SA node cell action potential depolarization [GO:0086041] Regulation: negatively regulated by negative regulation of voltage-gated potassium channel activity [GO:1903817]; positively regulated by GO:1903818